{
  "term_label": "proteolysis",
  "gene_name": "A disintegrin and metalloproteinase with thrombospondin motifs 19",
  "gene_symbol": "ADAMTS19",
  "gene": "UniProtKB:Q8TE59",
  "term_id": "GO:0006508"
}